{
  "gene_name": "Heme oxygenase 2",
  "gene": "UniProtKB:P30519",
  "term_id": "GO:0042167",
  "term_label": "heme catabolic process",
  "gene_symbol": "HMOX2"
}